symbiont-mediated suppression of host calcium-mediated signal transduction [GO:0075135] (BP) Also known as: disruption of host calcium or calmodulin-mediated signal transduction, negative regulation by symbiont of host Ca++ or calmodulin-mediated signal transduction, negative regulation by symbiont of host calcium or calmodulin-mediated signal transduction, suppression by symbiont of host calcium or calmodulin-mediated signal transduction, symbiont-mediated suppression of host calcium or calmodulin-mediated signal transduction Sources: GOC:pamgo_curators Definition: A process in which a symbiont interferes with, inhibits or disrupts a calcium signal transduction in the host organism. The host is defined as the larger of the organisms involved in a symbiotic interaction. Relationships: is_a GO:0052029